{
  "term_id": "UNKNOWN:0002",
  "gene_symbol": "CCDC182",
  "gene": "UniProtKB:A6NF36",
  "term_label": "Unknown biological process",
  "gene_name": "Coiled-coil domain-containing protein 182"
}